{
  "gene_symbol": "TMOD4",
  "term_label": "myofibril assembly",
  "gene_name": "Tropomodulin-4",
  "gene": "UniProtKB:Q9NZQ9",
  "term_id": "GO:0030239"
}